{
  "gene": "UniProtKB:Q9UKC9",
  "gene_symbol": "FBXL2",
  "term_id": "GO:0005737",
  "gene_name": "F-box_LRR-repeat protein 2",
  "term_label": "cytoplasm"
}